{
  "term_label": "developmental process",
  "term_id": "GO:0032502",
  "gene_name": "Twist-related protein 1",
  "gene_symbol": "TWIST1",
  "gene": "UniProtKB:Q15672"
}